{
  "term_label": "cytoplasm",
  "gene": "UniProtKB:Q13895",
  "gene_symbol": "BYSL",
  "term_id": "GO:0005737",
  "gene_name": "Bystin"
}